{
  "gene_symbol": "HS3ST6",
  "gene_name": "Heparan sulfate glucosamine 3-O-sulfotransferase 6",
  "term_label": "[heparan sulfate]-glucosamine 3-sulfotransferase activity",
  "term_id": "GO:0008467",
  "gene": "UniProtKB:Q96QI5"
}